{
  "gene_name": "Neuronal acetylcholine receptor subunit alpha-2",
  "gene_symbol": "CHRNA2",
  "gene": "UniProtKB:Q15822",
  "term_id": "GO:0022848",
  "term_label": "acetylcholine-gated monoatomic cation-selective channel activity"
}